regulation of low-density lipoprotein particle receptor catabolic process [GO:0032803] (biological process) Definition: Any process that modulates the frequency, rate or extent of the chemical reactions and pathways resulting in the breakdown of low-density lipoprotein particle receptors. Sources: GOC:mah Also known as: regulation of LDLr catabolic process, regulation of LDLr catabolism, regulation of low-density lipoprotein receptor breakdown, regulation of low-density lipoprotein receptor catabolic process, regulation of low-density lipoprotein receptor catabolism, regulation of low-density lipoprotein receptor degradation Relationships: is a type of regulation of protein catabolic process [GO:0042176]; is_a regulation of receptor catabolic process [GO:2000644]; regulates low-density lipoprotein particle receptor catabolic process [GO:0032802] Subtypes: negative regulation of low-density lipoprotein particle receptor catabolic process [GO:0032804], GO:0032805